negative regulation of all-trans-retinyl-ester hydrolase, 11-cis retinol forming activity [GO:0062003] (biological process) References: PMID:23407971 Definition: Any process that decreases the frequency or rate of all-trans-retinyl-ester hydrolase, 11-cis retinol forming activity. Relationships: is_a GO:0051346; is a type of negative regulation of small molecule metabolic process [GO:0062014]; RO_0002212 all-trans-retinyl-ester hydrolase, 11-cis retinol forming activity [GO:0052885]